{
  "term_label": "synaptic transmission, glutamatergic",
  "gene": "UniProtKB:P48058",
  "gene_name": "Glutamate receptor 4",
  "term_id": "GO:0035249",
  "gene_symbol": "GRIA4"
}